{
  "gene_symbol": "BOLA1",
  "gene": "UniProtKB:Q9Y3E2",
  "term_label": "Unknown biological process",
  "gene_name": "BolA-like protein 1",
  "term_id": "UNKNOWN:0002"
}